regulation of glucose mediated signaling pathway [GO:1902659] (biological process) References: PMID:24277933 Sources: GOC:TermGenie, GOC:di, GO_REF:0000058 Relationships: is a type of regulation of signal transduction [GO:0009966]; regulates glucose mediated signaling pathway [GO:0010255] Subtypes: regulation of adenylate cyclase-activating glucose-activated G protein-coupled receptor signaling pathway [GO:0110033], negative regulation of glucose mediated signaling pathway [GO:1902660], positive regulation of glucose mediated signaling pathway [GO:1902661] Also known as: regulation of glucose mediated signalling Definition: Any process that modulates the frequency, rate or extent of glucose mediated signaling pathway.